{
  "term_label": "vacuolar proton-transporting V-type ATPase complex",
  "term_id": "GO:0016471",
  "gene_name": "V-type proton ATPase 116 kDa subunit a 4",
  "gene_symbol": "ATP6V0A4",
  "gene": "UniProtKB:Q9HBG4"
}